{
  "gene_name": "EF-hand calcium-binding domain-containing protein 4B",
  "gene": "UniProtKB:Q9BSW2",
  "term_id": "UNKNOWN:0003",
  "gene_symbol": "CRACR2A",
  "term_label": "Unknown cellular component"
}